{
  "gene": "UniProtKB:Q96FQ6",
  "term_label": "extracellular space",
  "term_id": "GO:0005615",
  "gene_symbol": "S100A16",
  "gene_name": "Protein S100-A16"
}